{
  "gene": "UniProtKB:Q8WXE9",
  "term_id": "GO:0048488",
  "gene_symbol": "STON2",
  "term_label": "synaptic vesicle endocytosis",
  "gene_name": "Stonin-2"
}